{
  "term_id": "UNKNOWN:0001",
  "gene": "UniProtKB:Q5BKY9",
  "term_label": "Unknown molecular function",
  "gene_name": "Protein FAM133B",
  "gene_symbol": "FAM133B"
}